{
  "gene_name": "E3 ubiquitin-protein ligase XIAP",
  "gene_symbol": "XIAP",
  "gene": "UniProtKB:P98170",
  "term_label": "negative regulation of apoptotic process",
  "term_id": "GO:0043066"
}